negative regulation of glyoxylate cycle [GO:2000875] (biological process) Also known as: negative regulation of glyoxylate bypass Relationships: is a type of negative regulation of carbohydrate metabolic process [GO:0045912]; is a type of negative regulation of small molecule metabolic process [GO:0062014]; is a type of regulation of glyoxylate cycle [GO:2000874]; negatively regulates GO:0006097 Definition: Any process that stops, prevents or reduces the frequency, rate or extent of glyoxylate cycle. Sources: GOC:dgf